positive regulation of butyryl-CoA catabolic process to butanol [GO:1900499] (biological process) Also known as: activation of butyryl-CoA catabolism to butanol, positive regulation of butyryl-CoA catabolism to butanol, up regulation of butyryl-CoA catabolic process to butanol, up regulation of butyryl-CoA catabolism to butanol, up-regulation of butyryl-CoA catabolic process to butanol, up-regulation of butyryl-CoA catabolism to butanol, upregulation of butyryl-CoA catabolic process to butanol, upregulation of butyryl-CoA catabolism to butanol, activation of butyryl-CoA catabolic process to butanol Relationships: is a type of positive regulation of amide metabolic process [GO:0034250]; is_a positive regulation of fatty acid metabolic process [GO:0045923]; is a type of positive regulation of phosphate metabolic process [GO:0045937]; is a type of GO:0046889; is a type of positive regulation of lipid catabolic process [GO:0050996]; is a type of GO:1900497; is a type of positive regulation of alcohol biosynthetic process [GO:1902932]; positively regulates butyryl-CoA catabolic process to butanol [GO:0044582] Definition: Any process that activates or increases the frequency, rate or extent of butyryl-CoA catabolic process to butanol. Sources: GOC:TermGenie, GOC:mengo_curators